prenylcysteine methylesterase activity [GO:0010296] (molecular function) Relationships: is a type of protein methylesterase activity [GO:0051723] Definition: Catalysis of the reaction: protein C-terminal S-farnesyl-L-cysteine methyl ester + H2O = protein C-terminal S-farnesyl-L-cysteine + methanol + H+. References: PMID:16870359 Sources: RHEA:48520